{
  "term_label": "Unknown molecular function",
  "gene": "UniProtKB:Q9UBC7",
  "gene_symbol": "GALP",
  "gene_name": "Galanin-like peptide",
  "term_id": "UNKNOWN:0001"
}